{
  "gene": "UniProtKB:P25090",
  "term_id": "GO:0007204",
  "gene_name": "N-formyl peptide receptor 2",
  "term_label": "positive regulation of cytosolic calcium ion concentration",
  "gene_symbol": "FPR2"
}